dibenzothiophene sulfone monooxygenase (NADH) activity [GO:0018679] (molecular function) Sources: RHEA:12312 Definition: Catalysis of the reaction: dibenzothiophene 5,5-dioxide + FMNH2 + NADH + O2 = 2'-hydroxybiphenyl-2-sulfinate + FMN + H+ + H2O + NAD+. Also known as: dibenzothiophene-5,5-dioxide monooxygenase activity Relationships: is a type of GO:0016712